{
  "gene": "UniProtKB:Q66K14",
  "term_id": "UNKNOWN:0003",
  "term_label": "Unknown cellular component",
  "gene_symbol": "TBC1D9B",
  "gene_name": "TBC1 domain family member 9B"
}